{
  "term_id": "GO:0000978",
  "gene_symbol": "FOXL2",
  "gene": "UniProtKB:P58012",
  "term_label": "RNA polymerase II cis-regulatory region sequence-specific DNA binding",
  "gene_name": "Forkhead box protein L2"
}